{
  "gene_name": "DNA repair protein RAD51 homolog 1",
  "term_id": "GO:0000730",
  "gene": "UniProtKB:Q06609",
  "term_label": "DNA recombinase assembly",
  "gene_symbol": "RAD51"
}